{
  "term_id": "GO:0006355",
  "gene": "UniProtKB:Q9NZR4",
  "gene_name": "Visual system homeobox 1",
  "gene_symbol": "VSX1",
  "term_label": "regulation of DNA-templated transcription"
}